{
  "gene_symbol": "BARX2",
  "gene": "UniProtKB:Q9UMQ3",
  "gene_name": "Homeobox protein BarH-like 2",
  "term_id": "GO:0006357",
  "term_label": "regulation of transcription by RNA polymerase II"
}